2-acetolactate mutase activity [GO:0047534] (MF) Definition: Catalysis of the reaction: 2-acetolactate = 3-hydroxy-3-methyl-2-oxobutanoate. Sources: EC:5.4.99.3, MetaCyc:2-ACETOLACTATE-MUTASE-RXN Relationships: is a type of intramolecular transferase activity [GO:0016866] Also known as: acetohydroxy acid isomerase activity, 2-acetolactate methylmutase activity, acetolactate mutase activity